{
  "term_label": "site of double-strand break",
  "gene": "UniProtKB:P49959",
  "term_id": "GO:0035861",
  "gene_symbol": "MRE11",
  "gene_name": "Double-strand break repair protein MRE11"
}